{
  "gene_name": "Lysosomal alpha-glucosidase",
  "gene_symbol": "GAA",
  "gene": "UniProtKB:P10253",
  "term_id": "GO:0007040",
  "term_label": "lysosome organization"
}